{
  "gene_name": "Protein lin-7 homolog A",
  "term_label": "cell-cell junction",
  "gene": "UniProtKB:O14910",
  "gene_symbol": "LIN7A",
  "term_id": "GO:0005911"
}